{
  "gene_symbol": "TMEM106A",
  "term_id": "UNKNOWN:0002",
  "gene": "UniProtKB:Q96A25",
  "term_label": "Unknown biological process",
  "gene_name": "Transmembrane protein 106A"
}